release of cytochrome c from mitochondria [GO:0001836] (biological process) Definition: The process that results in the movement of cytochrome c from the mitochondrial intermembrane space into the cytosol, which is part of the apoptotic signaling pathway and leads to caspase activation. References: PMID:12925707, PMID:9560217 Sources: GOC:add, GOC:mah, GOC:mtg_apoptosis, ISBN:0721639976 Note: The release of cytochrome c from mitochondria is a central event in the signaling phase of the apoptotic process, and it is often used by researchers to monitor this type of cell death. Any event that induces apoptosis will at some point induce the release of cytochrome c from mitochondria. Therefore, this term should only be used to annotate gene products that are directly involved in this process. An example is Drp1 (DNM1L, UniProt symbol O00429) in PMID:20850011. Relationships: is a type of apoptotic mitochondrial changes [GO:0008637]; is part of apoptotic signaling pathway [GO:0097190] Regulation: regulated by regulation of release of cytochrome c from mitochondria [GO:0090199]; positively regulated by positive regulation of release of cytochrome c from mitochondria [GO:0090200]; negatively regulated by negative regulation of release of cytochrome c from mitochondria [GO:0090201]